echolocation [GO:0050959] (biological process) Relationships: is a type of nervous system process [GO:0050877] References: PMID:16005275 Sources: Wikipedia:Animal_echolocation Also known as: biological sonar, perception of environment using reflected sound waves Definition: Echolocation is the method used by some animals (e.g. bats, dolphins and some whales) to determine the location of something by measuring the time it takes for an echo to return from it. These animals emit sound waves and listen for the echo, calculating the distance to the object from the time lapse between sound emission and the echo returning.